cortical microtubule cytoskeleton [GO:0030981] (cellular component) Sources: GOC:mah Definition: The portion of the microtubule cytoskeleton that lies just beneath the plasma membrane. Relationships: is a type of cortical cytoskeleton [GO:0030863]; is part of microtubule cytoskeleton [GO:0015630]